{
  "gene_name": "Disintegrin and metalloproteinase domain-containing protein 17",
  "term_id": "GO:0004222",
  "gene": "UniProtKB:P78536",
  "term_label": "metalloendopeptidase activity",
  "gene_symbol": "ADAM17"
}